regulation of Malpighian tubule diameter [GO:0035297] (biological process) References: PMID:9286684 Relationships: is a type of regulation of tube diameter [GO:0035296]; is a type of regulation of Malpighian tubule size [GO:0035298] Definition: Ensuring that the Malpighian tubule is the correct width. Malpighian tubules have a uniform circumference along their length; the circumference of the tubes is eight cells during the time the cells are dividing, after which the cells rearrange producing tubes with a cirumference of two cells.